{
  "gene": "UniProtKB:Q9Y2I7",
  "term_id": "GO:0000285",
  "term_label": "1-phosphatidylinositol-3-phosphate 5-kinase activity",
  "gene_name": "1-phosphatidylinositol 3-phosphate 5-kinase",
  "gene_symbol": "PIKFYVE"
}